transcription elongation factor activity [GO:0003711] (molecular function) Relationships: is a type of transcription regulator activity [GO:0140110] Note: Restored term from obsolete. References: PMID:23878398, PMID:28892040 Sources: GOC:txnOH-2018 Also known as: transcription elongation regulator activity, transcriptional elongation regulator activity Definition: A molecular function that stimulates the elongation properties of the RNA polymerase during the elongation phase of transcription. A subclass of transcription elongation factors enable the transition from transcription initiation to elongation, while another class rescue stalled RNA polymerases.